{
  "gene": "UniProtKB:Q9P0S2",
  "gene_name": "Cytochrome c oxidase assembly protein COX16 homolog, mitochondrial",
  "term_id": "GO:0005743",
  "term_label": "mitochondrial inner membrane",
  "gene_symbol": "COX16"
}